{
  "gene_symbol": "BANF1",
  "gene_name": "Barrier-to-autointegration factor",
  "term_id": "GO:0051276",
  "term_label": "chromosome organization",
  "gene": "UniProtKB:O75531"
}